{
  "gene_name": "LIM domain-containing protein ajuba",
  "gene_symbol": "AJUBA",
  "gene": "UniProtKB:Q96IF1",
  "term_label": "response to hypoxia",
  "term_id": "GO:0001666"
}